poly-pyrimidine tract binding [GO:0008187] (molecular function) Sources: GOC:jl Relationships: is a type of GO:0003727 Definition: Binding to a stretch of pyrimidines (cytosine or uracil) in an RNA molecule. Subtypes: poly(U) RNA binding [GO:0008266], poly(C) RNA binding [GO:0017130], uridine-rich cytoplasmic polyadenylylation element binding [GO:0017131]